{
  "gene_symbol": "SEC61A2",
  "term_id": "GO:0006616",
  "gene_name": "Protein transport protein Sec61 subunit alpha isoform 2",
  "term_label": "SRP-dependent cotranslational protein targeting to membrane, translocation",
  "gene": "UniProtKB:Q9H9S3"
}